2-methylbutanoate-CoA ligase activity [GO:0043759] (molecular function) Relationships: is a type of short-chain fatty acid-CoA ligase activity [GO:0031955] Sources: RHEA:46180 Definition: Catalysis of the reaction: ATP + 2-methylbutanoate + CoA = AMP + diphosphate + 2-methylbutanoyl-CoA. Also known as: branched chain acyl CoA synthetase (ADP-forming) activity, branched chain acyl-CoA synthetase (ADP-forming) activity, branched-chain acyl CoA synthetase (ADP-forming) activity, branched-chain acyl-CoA synthetase (ADP-forming) activity